{
  "gene": "UniProtKB:Q99457",
  "gene_name": "Nucleosome assembly protein 1-like 3",
  "term_id": "GO:0006334",
  "gene_symbol": "NAP1L3",
  "term_label": "nucleosome assembly"
}